{
  "gene": "UniProtKB:P09067",
  "term_id": "GO:0006357",
  "gene_name": "Homeobox protein Hox-B5",
  "term_label": "regulation of transcription by RNA polymerase II",
  "gene_symbol": "HOXB5"
}